hormone secretion [GO:0046879] (biological process) Subtypes: histamine secretion involved in inflammatory response [GO:0002441], peptide hormone secretion [GO:0030072], activin secretion [GO:0032333], GO:0035936, androstenedione secretion [GO:0035941], dehydroepiandrosterone secretion [GO:0035942], endocrine hormone secretion [GO:0060986] Definition: The regulated release of hormones, substances with a specific regulatory effect on a particular organ or group of cells. Regulation: regulated by GO:0046883; RO_0002213 by positive regulation of hormone secretion [GO:0046887]; negatively regulated by GO:0046888 Sources: ISBN:0198506732 Relationships: is a type of GO:0009914; is a type of signal release [GO:0023061]